modification of dendritic spine [GO:0098886] (BP) Definition: Any process that modifies the structure of a dendritic spine. Relationships: is a type of modification of postsynaptic structure [GO:0099010] Note: This class does not cover assembly or disassembly of dendritic spines, only the modification/remodelling of existing ones. Sources: GOC:dos